{
  "gene": "UniProtKB:A8MX19",
  "gene_symbol": "FAM90A12P",
  "term_id": "UNKNOWN:0001",
  "term_label": "Unknown molecular function",
  "gene_name": "Putative protein FAM90A12P"
}